{
  "gene_symbol": "SFPQ",
  "gene": "UniProtKB:P23246",
  "term_label": "RNA binding",
  "term_id": "GO:0003723",
  "gene_name": "Splicing factor, proline- and glutamine-rich"
}